T=13 icosahedral viral capsid [GO:0039621] (cellular component) Definition: The protein coat that surrounds the infective nucleic acid in some virus particles where the subunits (capsomeres) are arranged to form an icosahedron with T=13 symmetry. The T=13 capsid is composed of 12 pentameric and 120 hexameric capsomeres. Relationships: is a type of icosahedral viral capsid [GO:0019030] Sources: VZ:260